{
  "gene_symbol": "CPEB1",
  "gene": "UniProtKB:Q9BZB8",
  "term_label": "neuron projection",
  "term_id": "GO:0043005",
  "gene_name": "Cytoplasmic polyadenylation element-binding protein 1"
}